{
  "term_id": "GO:0003724",
  "term_label": "RNA helicase activity",
  "gene": "UniProtKB:O00148",
  "gene_name": "ATP-dependent RNA helicase DDX39A",
  "gene_symbol": "DDX39A"
}